{
  "gene_symbol": "BBS7",
  "term_label": "axoneme",
  "gene": "UniProtKB:Q8IWZ6",
  "term_id": "GO:0005930",
  "gene_name": "Bardet-Biedl syndrome 7 protein"
}